{
  "gene": "UniProtKB:Q9H379",
  "term_id": "UNKNOWN:0002",
  "gene_symbol": "PRO3102",
  "term_label": "Unknown biological process",
  "gene_name": "Putative uncharacterized protein PRO3102"
}